{
  "gene_symbol": "GAS2L3",
  "term_id": "GO:0051764",
  "gene": "UniProtKB:Q86XJ1",
  "term_label": "actin crosslink formation",
  "gene_name": "GAS2-like protein 3"
}